{
  "term_label": "alpha-amylase activity",
  "gene_name": "Alpha-amylase 2B",
  "gene_symbol": "AMY2B",
  "gene": "UniProtKB:P19961",
  "term_id": "GO:0004556"
}